{
  "term_label": "DNA-binding transcription factor activity, RNA polymerase II-specific",
  "term_id": "GO:0000981",
  "gene_name": "Double homeobox protein 5",
  "gene": "UniProtKB:Q96PT3",
  "gene_symbol": "DUX5"
}